{
  "term_id": "GO:0043161",
  "gene_name": "Glucose-induced degradation protein 4 homolog",
  "term_label": "proteasome-mediated ubiquitin-dependent protein catabolic process",
  "gene_symbol": "GID4",
  "gene": "UniProtKB:Q8IVV7"
}